{
  "term_label": "Cul4-RING E3 ubiquitin ligase complex",
  "term_id": "GO:0080008",
  "gene_symbol": "DCAF8",
  "gene_name": "DDB1- and CUL4-associated factor 8",
  "gene": "UniProtKB:Q5TAQ9"
}